{
  "term_id": "UNKNOWN:0002",
  "gene_name": "tRNA-splicing endonuclease subunit Sen15",
  "term_label": "Unknown biological process",
  "gene": "UniProtKB:Q8WW01",
  "gene_symbol": "TSEN15"
}